regulation of termination of mating projection growth [GO:0031385] (biological process) Definition: Any process that modulates the frequency, rate, or extent of the end of mating projection formation by unicellular fungi. Relationships: is a type of regulation of mating projection assembly [GO:0031383] References: PMID:14734532